regulation of cell proliferation involved in embryonic placenta development [GO:0060723] (biological process) Sources: GOC:dph Subtypes: regulation of spongiotrophoblast cell proliferation [GO:0060721] Definition: Any process that modulates the rate, frequency, or extent of cell proliferation involved in embryonic placenta development. Relationships: is a type of regulation of cell population proliferation [GO:0042127]; regulates cell proliferation involved in embryonic placenta development [GO:0060722]